sorbitol transmembrane transport [GO:0015795] (biological process) Also known as: sorbitol transport, glucitol transport Sources: GOC:ai, ISBN:0198506732 Definition: The directed movement of sorbitol across a membrane. Sorbitol, also known as glucitol, is the hexitol derived by the reduction of the aldehyde group of glucose. Relationships: is a type of polyol transmembrane transport [GO:0015791]; is a type of carbohydrate transmembrane transport [GO:0034219]